{
  "term_id": "UNKNOWN:0001",
  "gene": "UniProtKB:Q92917",
  "gene_symbol": "GPKOW",
  "term_label": "Unknown molecular function",
  "gene_name": "G-patch domain and KOW motifs-containing protein"
}